{
  "gene_name": "Probable E3 ubiquitin-protein ligase HECTD2",
  "term_id": "UNKNOWN:0003",
  "gene": "UniProtKB:Q5U5R9",
  "term_label": "Unknown cellular component",
  "gene_symbol": "HECTD2"
}